pheromone response MAPK cascade [GO:0071507] (biological process) References: PMID:17604854 Sources: GOC:mah, GOC:vw Definition: A MAPK cascade containing at least the Fus3 MAP kinase. It starts with the activation of Ste20, a MAP4K, which activates Ste11, a MAP3K, which in turn activate Ste7, a MAP2K, which activates Fus3. The kinases in each tier phosphorylate and activate the kinases in the downstream tier. This MAPK cascade is triggered by a pheromone activating its G protein-coupled receptor, and results in cellular responses that lead to conjugation with cellular fusion. Relationships: is a type of MAPK cascade [GO:0000165]; is part of conjugation with cellular fusion [GO:0000747]; is part of pheromone-dependent signal transduction involved in conjugation with cellular fusion [GO:0000750] Regulation: positively regulated by GO:0062038; regulated by regulation of pheromone response MAPK cascade [GO:0180039]; negatively regulated by negative regulation of pheromone response MAPK cascade [GO:0180040] Also known as: MAPK cascade involved in conjugation with cellular fusion, MAPKKK cascade involved in conjugation with cellular fusion, conjugation with cellular fusion, MAPKKK cascade, Fus3 signaling cascade, MAPK signaling in response to pheromone, MAPKKK cascade involved in mating response, pheromone MAPK module